{
  "term_label": "motile cilium",
  "gene_name": "IQ and ubiquitin-like domain-containing protein",
  "term_id": "GO:0031514",
  "gene_symbol": "IQUB",
  "gene": "UniProtKB:Q8NA54"
}